{
  "gene_symbol": "S100B",
  "gene": "UniProtKB:P04271",
  "gene_name": "Protein S100-B",
  "term_id": "GO:0008284",
  "term_label": "positive regulation of cell population proliferation"
}